{
  "gene_name": "Reticulon-4 receptor",
  "term_id": "GO:1905576",
  "term_label": "ganglioside GT1b binding",
  "gene": "UniProtKB:Q9BZR6",
  "gene_symbol": "RTN4R"
}